{
  "term_label": "Unknown cellular component",
  "term_id": "UNKNOWN:0003",
  "gene_symbol": "ILF3",
  "gene": "UniProtKB:Q12906",
  "gene_name": "Interleukin enhancer-binding factor 3"
}